{
  "gene_symbol": "CFHR4",
  "term_id": "GO:0005615",
  "gene_name": "Complement factor H-related protein 4",
  "term_label": "extracellular space",
  "gene": "UniProtKB:Q92496"
}